{
  "term_label": "phosphatidylinositol dephosphorylation",
  "gene": "UniProtKB:Q13613",
  "gene_symbol": "MTMR1",
  "gene_name": "Myotubularin-related protein 1",
  "term_id": "GO:0046856"
}